nuclear matrix organization [GO:0043578] (biological process) Sources: GOC:dph, GOC:jl, GOC:mah Definition: A process that is carried out at the cellular level which results in the assembly, arrangement of constituent parts, or disassembly of the nuclear matrix, the dense fibrillar network lying on the inner side of the nuclear membrane. Also known as: nuclear matrix organisation, nucleoskeleton organization, nuclear matrix organization and biogenesis Relationships: is a type of GO:0006997 Subtypes: nuclear matrix anchoring at nuclear membrane [GO:0090292]